MWP complex [GO:1990811] (cellular component) Definition: A protein ternary complex that anchors microtubule minus ends to mitotic spindle pole bodies. The founding complex contains a microtubule anchoring protein (Msd1 in fission yeast), A WD-repeat Wdr8 family protein and and a minus end-directed kinesin. Also known as: Msd1-Wdr8-Pkl1 complex Relationships: is a type of protein-containing complex [GO:0032991] References: PMID:25987607, PMID:29021344